{
  "term_label": "Unknown molecular function",
  "gene": "UniProtKB:A0A0U1RRL7",
  "gene_symbol": "MMP24OS",
  "term_id": "UNKNOWN:0001",
  "gene_name": "Protein MMP24OS"
}